{
  "gene_name": "Putative histone H2B type 2-C",
  "term_label": "antimicrobial humoral immune response mediated by antimicrobial peptide",
  "gene_symbol": "H2BC20P",
  "gene": "UniProtKB:Q6DN03",
  "term_id": "GO:0061844"
}